purine nucleoside diphosphate catabolic process [GO:0009137] (biological process) Definition: The chemical reactions and pathways resulting in the breakdown of purine nucleoside diphosphate, a compound consisting of a purine base linked to a ribose or deoxyribose sugar esterified with diphosphate on the sugar. Sources: GOC:go_curators, ISBN:0198506732 Also known as: purine nucleoside diphosphate breakdown, purine nucleoside diphosphate catabolism, purine nucleoside diphosphate degradation Relationships: is a type of nucleoside diphosphate catabolic process [GO:0009134]; is a type of purine nucleoside diphosphate metabolic process [GO:0009135] Subtypes: purine ribonucleoside diphosphate catabolic process [GO:0009181], purine deoxyribonucleoside diphosphate catabolic process [GO:0009184]